{
  "gene_name": "1-phosphatidylinositol 4,5-bisphosphate phosphodiesterase beta-2",
  "term_id": "GO:0007186",
  "gene_symbol": "PLCB2",
  "gene": "UniProtKB:Q00722",
  "term_label": "G protein-coupled receptor signaling pathway"
}